{
  "gene": "UniProtKB:O95237",
  "gene_symbol": "LRAT",
  "gene_name": "Lecithin retinol acyltransferase",
  "term_label": "vitamin A metabolic process",
  "term_id": "GO:0006776"
}